{
  "term_label": "N-acetylglucosamine metabolic process",
  "gene": "UniProtKB:Q9GZS9",
  "gene_name": "Carbohydrate sulfotransferase 5",
  "gene_symbol": "CHST5",
  "term_id": "GO:0006044"
}